{
  "term_id": "GO:0005737",
  "term_label": "cytoplasm",
  "gene_name": "Sulfotransferase 1C2",
  "gene": "UniProtKB:O00338",
  "gene_symbol": "SULT1C2"
}